{
  "term_label": "zinc chaperone activity",
  "term_id": "GO:0140827",
  "gene_symbol": "ZNG1E",
  "gene": "UniProtKB:Q5RIA9",
  "gene_name": "Zinc-regulated GTPase metalloprotein activator 1E"
}